4-hydroxy-tetrahydrodipicolinate reductase [GO:0008839] (molecular function) Relationships: is a type of oxidoreductase activity, acting on the CH-CH group of donors, NAD or NADP as acceptor [GO:0016628] Sources: EC:1.17.1.8 Definition: Catalysis of the reaction: (S)-2,3,4,5-tetrahydropyridine-2,6-dicarboxylate + NAD(P)+ + H2O = (2S,4S)-4-hydroxy-2,3,4,5-tetrahydrodipicolinate + NAD(P)H + H+. Also known as: dihydrodipicolinate reductase activity, 2,3,4,5-tetrahydrodipicolinate:NAD(P)+ oxidoreductase activity, dihydrodipicolinic acid reductase activity